NF-kappaB binding [GO:0051059] (molecular function) Definition: Binding to NF-kappaB, a transcription factor for eukaryotic RNA polymerase II promoters. Sources: GOC:ai Relationships: is_a RNA polymerase II-specific DNA-binding transcription factor binding [GO:0061629]